{
  "gene": "UniProtKB:P55017",
  "gene_symbol": "SLC12A3",
  "gene_name": "Solute carrier family 12 member 3",
  "term_id": "GO:1990573",
  "term_label": "potassium ion import across plasma membrane"
}